regulation of cilium beat frequency involved in ciliary motility [GO:0060296] (biological process) Relationships: is a type of regulation of cilium beat frequency [GO:0003356]; is a type of GO:0060295; is a type of regulation of biological quality [GO:0065008] Definition: Any process that modulates the frequency of cilium beating involved in ciliary motility. Subtypes: positive regulation of cilium beat frequency involved in ciliary motility [GO:0120030] Sources: GOC:BHF, GOC:cilia, GOC:dph, GOC:krc, GOC:tb